{
  "gene_symbol": "PLK1",
  "gene_name": "Serine_threonine-protein kinase PLK1",
  "term_label": "nucleus",
  "term_id": "GO:0005634",
  "gene": "UniProtKB:P53350"
}